{
  "gene": "UniProtKB:P35241",
  "gene_name": "Radixin",
  "term_label": "apical part of cell",
  "gene_symbol": "RDX",
  "term_id": "GO:0045177"
}